{
  "gene": "UniProtKB:Q9BQQ3",
  "term_id": "GO:0007030",
  "term_label": "Golgi organization",
  "gene_symbol": "GORASP1",
  "gene_name": "Golgi reassembly-stacking protein 1"
}